{
  "term_label": "RNA binding",
  "gene_name": "Large ribosomal subunit protein eL14",
  "gene": "UniProtKB:P50914",
  "gene_symbol": "RPL14",
  "term_id": "GO:0003723"
}